positive regulation of aspartate secretion [GO:1904450] (biological process) Relationships: is a type of positive regulation of organic acid transport [GO:0032892]; is a type of GO:0051957; is a type of positive regulation of secretion by cell [GO:1903532]; is a type of regulation of aspartate secretion [GO:1904448]; positively regulates aspartate secretion [GO:0061528] References: PMID:2342602 Sources: GOC:TermGenie, GO_REF:0000058 Definition: Any process that activates or increases the frequency, rate or extent of aspartate secretion. Also known as: up regulation of aspartate secretion, up-regulation of aspartate secretion, upregulation of aspartate secretion, activation of aspartate secretion